{
  "gene_symbol": "OR14K1",
  "term_id": "GO:0004984",
  "term_label": "olfactory receptor activity",
  "gene_name": "Olfactory receptor 14K1",
  "gene": "UniProtKB:Q8NGZ2"
}